{
  "term_id": "UNKNOWN:0003",
  "term_label": "Unknown cellular component",
  "gene_symbol": "PSORS1C1",
  "gene_name": "Psoriasis susceptibility 1 candidate gene 1 protein",
  "gene": "UniProtKB:Q9UIG5"
}